{
  "gene_symbol": "RC3H2",
  "term_id": "GO:0006511",
  "gene_name": "Roquin-2",
  "term_label": "ubiquitin-dependent protein catabolic process",
  "gene": "UniProtKB:Q9HBD1"
}